cysteine transmembrane transporter activity [GO:0033229] (MF) Subtypes: GO:0033230 Sources: GOC:mah Relationships: is a type of GO:0000099; is a type of neutral L-amino acid transmembrane transporter activity [GO:0015175]; is part of cysteine transmembrane transport [GO:1903712] Definition: Enables the transfer of cysteine from one side of a membrane to the other.